{
  "term_label": "Unknown molecular function",
  "gene_symbol": "THOC1",
  "gene_name": "THO complex subunit 1",
  "term_id": "UNKNOWN:0001",
  "gene": "UniProtKB:Q96FV9"
}